{
  "term_id": "GO:0035627",
  "gene_name": "Ceramide-1-phosphate transfer protein",
  "gene_symbol": "CPTP",
  "gene": "UniProtKB:Q5TA50",
  "term_label": "ceramide transport"
}